estrogen metabolic process [GO:0008210] (biological process) Definition: The chemical reactions and pathways involving estrogens, C18 steroid hormones that can stimulate the development of female sexual characteristics. Also found in plants. Sources: ISBN:0198506732 Relationships: is a type of steroid metabolic process [GO:0008202]; is_a GO:0042445 Subtypes: estrogen biosynthetic process [GO:0006703], GO:0006711 Also known as: estrogen metabolism, oestrogen metabolic process, oestrogen metabolism